{
  "gene_symbol": "PRR35",
  "gene_name": "Proline-rich protein 35",
  "term_id": "UNKNOWN:0002",
  "gene": "UniProtKB:P0CG20",
  "term_label": "Unknown biological process"
}